{
  "term_id": "UNKNOWN:0001",
  "gene_name": "Putative uncharacterized protein FLJ13197",
  "term_label": "Unknown molecular function",
  "gene_symbol": "Q9H8V8",
  "gene": "UniProtKB:Q9H8V8"
}